plasmanylethanolamine desaturase activity [GO:0050207] (MF) Relationships: is a type of oxidoreductase activity, acting on paired donors, with oxidation of a pair of donors resulting in the reduction of molecular oxygen to two molecules of water [GO:0016717] Definition: Catalysis of the reaction:1-(1,2-saturated alkyl)-2-acyl-sn-glycero-3-phosphoethanolamine + 2 Fe(II)-[cytochrome b5] + 2 H+ + O2 = 1-O-(1Z-alkenyl)-2-acyl-sn-glycero-3-phosphoethanolamine + 2 Fe(III)-[cytochrome b5] + 2 H2O. Sources: RHEA:22956 Also known as: plasmenylethanolamine desaturase activity, 2-acyl-1-alkyl-sn-glycero-3-phosphoethanolamine desaturase activity, alkylacylglycero-phosphorylethanolamine dehydrogenase activity, alkylacylglycerophosphoethanolamine desaturase activity